positive regulation of macrophage chemotaxis [GO:0010759] (biological process) Definition: Any process that increases the rate, frequency or extent of macrophage chemotaxis. Macrophage chemotaxis is the movement of a macrophage in response to an external stimulus. Sources: GOC:BHF, GOC:dph, GOC:tb Relationships: is a type of GO:0002690; is a type of regulation of macrophage chemotaxis [GO:0010758]; is a type of regulation of granulocyte chemotaxis [GO:0071622]; is a type of positive regulation of macrophage migration [GO:1905523]; positively regulates macrophage chemotaxis [GO:0048246]